viral latency [GO:0019042] (biological process) Sources: GOC:jl, VZ:3970 Also known as: latent virus infection, phage lysogeny, viral dormancy Definition: The process by which, after initial infection, a virus lies dormant within a cell and viral production ceases. The process ends when the virus switches from latency and starts to replicate. Relationships: is a type of GO:0016032